histone H4 ubiquitin ligase activity [GO:0141056] (molecular function) References: PMID:25303536 Definition: Catalysis of the transfer of ubiquitin to a histone H4 substrate. Subtypes: GO:0141000 Relationships: is a type of histone ubiquitin ligase activity [GO:0140852]